telomere single strand break repair [GO:1903823] (biological process) Regulation: negatively regulated by GO:1903824 Definition: Single strand break repair that takes place in a telomere. Relationships: is a type of single strand break repair [GO:0000012]; occurs in chromosome, telomeric region [GO:0000781] References: PMID:24374808 Sources: GOC:TermGenie, GO_REF:0000062 Also known as: single strand break repair in telomere, telomere single-strand break repair, telomeric single strand break repair, telomere SSBR